{
  "gene_name": "Pumilio homolog 2",
  "gene": "UniProtKB:Q8TB72",
  "term_id": "GO:0035196",
  "term_label": "miRNA processing",
  "gene_symbol": "PUM2"
}